{
  "gene_name": "Sperm protein associated with the nucleus on the X chromosome N5",
  "gene": "UniProtKB:Q5MJ07",
  "term_id": "UNKNOWN:0003",
  "term_label": "Unknown cellular component",
  "gene_symbol": "SPANXN5"
}